{
  "gene": "UniProtKB:P50226",
  "gene_name": "Sulfotransferase 1A2",
  "gene_symbol": "SULT1A2",
  "term_id": "GO:0051923",
  "term_label": "sulfation"
}